{
  "term_label": "clathrin binding",
  "gene_symbol": "EPN2",
  "gene": "UniProtKB:O95208",
  "gene_name": "Epsin-2",
  "term_id": "GO:0030276"
}